{
  "gene": "UniProtKB:Q8N2Q7",
  "term_id": "GO:0099634",
  "term_label": "postsynaptic specialization membrane",
  "gene_name": "Neuroligin-1",
  "gene_symbol": "NLGN1"
}